{
  "gene_symbol": "EVA1A",
  "term_label": "Unknown biological process",
  "gene_name": "Protein eva-1 homolog A",
  "term_id": "UNKNOWN:0002",
  "gene": "UniProtKB:Q9H8M9"
}